{
  "term_id": "GO:0005634",
  "gene_symbol": "SRA1",
  "term_label": "nucleus",
  "gene": "UniProtKB:Q9HD15",
  "gene_name": "Steroid receptor RNA activator 1"
}